{
  "term_label": "condensed chromosome",
  "gene": "UniProtKB:Q9H503",
  "term_id": "GO:0000793",
  "gene_name": "Barrier-to-autointegration factor-like protein",
  "gene_symbol": "BANF2"
}